{
  "term_id": "GO:0006954",
  "gene_symbol": "PYCARD",
  "gene_name": "Apoptosis-associated speck-like protein containing a CARD",
  "term_label": "inflammatory response",
  "gene": "UniProtKB:Q9ULZ3"
}